{
  "gene": "UniProtKB:P38435",
  "gene_symbol": "GGCX",
  "term_label": "Unknown cellular component",
  "term_id": "UNKNOWN:0003",
  "gene_name": "Vitamin K-dependent gamma-carboxylase"
}